{
  "gene": "UniProtKB:Q6ZUT1",
  "gene_name": "Uncharacterized protein NKAPD1",
  "term_label": "Unknown biological process",
  "term_id": "UNKNOWN:0002",
  "gene_symbol": "NKAPD1"
}